negative regulation of cell proliferation in bone marrow [GO:1903769] (biological process) Definition: Any process that stops, prevents or reduces the frequency, rate or extent of cell proliferation in bone marrow. Relationships: is a type of negative regulation of cell population proliferation [GO:0008285]; is a type of regulation of cell proliferation in bone marrow [GO:0071863]; negatively regulates GO:0071838 Also known as: down regulation of bone marrow cell proliferation, down regulation of cell proliferation in bone marrow, down-regulation of bone marrow cell proliferation, down-regulation of cell proliferation in bone marrow, downregulation of bone marrow cell proliferation, downregulation of cell proliferation in bone marrow, negative regulation of bone marrow cell proliferation, inhibition of bone marrow cell proliferation, inhibition of cell proliferation in bone marrow References: PMID:9241534 Sources: GOC:TermGenie, GO_REF:0000058